L-idonate transmembrane transport [GO:0015726] (biological process) Definition: The process in which L-idonate is transported across a lipid bilayer, from one side of a membrane to the other. L-idonate is an aldonic acid derived from L-idose, an aldohexose which is epimeric with D-glucose. Relationships: is a type of carbohydrate transmembrane transport [GO:0034219]; is a type of GO:0042873 Also known as: L-idonate transport Sources: GOC:krc